response to carboplatin [GO:0097328] (biological process) Definition: Any process that results in a change in state or activity of a cell or an organism (in terms of movement, secretion, enzyme production, gene expression, etc.) as a result of a carboplatin stimulus. Sources: GOC:pr Relationships: is a type of response to chemical [GO:0042221]